methionine transmembrane transporter activity [GO:0043865] (MF) Also known as: methionine importer activity, methionine importing activity, methionine-importing activity, methionine importer Relationships: is_a sulfur amino acid transmembrane transporter activity [GO:0000099]; is a type of amino acid transmembrane transporter activity [GO:0015171]; is part of GO:0015821 Subtypes: L-methionine transmembrane transporter activity [GO:0015191], ABC-type D-methionine transporter activity [GO:0033232] Definition: Enables the transfer of methionine from one side of a membrane to the other. Sources: GOC:jl